establishment of blood-brain barrier [GO:0060856] (biological process) Subtypes: establishment of endothelial blood-brain barrier [GO:0014045], establishment of glial blood-brain barrier [GO:0060857] Also known as: establishment of BBB, establishment of blood/brain barrier Definition: Establishment of the barrier between the blood and the brain. The cells in the brain are packed tightly together preventing the passage of most molecules from the blood into the brain. Only lipid soluble molecules or those that are actively transported can pass through the blood-brain barrier. Relationships: is a type of cell development [GO:0048468]; is part of central nervous system development [GO:0007417] Regulation: regulated by GO:0090210; positively regulated by positive regulation of establishment of blood-brain barrier [GO:0090211]; RO_0002212 by negative regulation of establishment of blood-brain barrier [GO:0090212] References: PMID:20080302, PMID:30280653 Sources: GOC:aruk, GOC:dph, GOC:sart